{
  "term_label": "Unknown biological process",
  "term_id": "UNKNOWN:0002",
  "gene_name": "Growth hormone-regulated TBC protein 1",
  "gene": "UniProtKB:Q5TC63",
  "gene_symbol": "GRTP1"
}